nurse cell nucleus anchoring [GO:0007302] (biological process) Sources: ISBN:0879694238 Definition: Attachment of the nurse cell nucleus to the plasma membrane. Relationships: is a type of nucleus localization [GO:0051647]